{
  "term_label": "endoplasmic reticulum",
  "gene_symbol": "P4HTM",
  "term_id": "GO:0005783",
  "gene": "UniProtKB:Q9NXG6",
  "gene_name": "Transmembrane prolyl 4-hydroxylase"
}